{
  "gene_symbol": "BTBD1",
  "gene_name": "BTB_POZ domain-containing protein 1",
  "term_id": "GO:0000932",
  "gene": "UniProtKB:Q9H0C5",
  "term_label": "P-body"
}